{
  "gene_symbol": "SMLR1",
  "gene": "UniProtKB:H3BR10",
  "term_id": "UNKNOWN:0003",
  "term_label": "Unknown cellular component",
  "gene_name": "Small leucine-rich protein 1"
}